{
  "term_id": "UNKNOWN:0002",
  "gene": "UniProtKB:Q685J3",
  "gene_name": "Mucin-17",
  "term_label": "Unknown biological process",
  "gene_symbol": "MUC17"
}